vesicle scission involved in endocytosis [GO:0099051] (biological process) Definition: The membrane scission process that is the final step in the formation of an endocytic vesicle: separation from the plasma membrane. Subtypes: vesicle scission involved in clathrin-mediated endocytosis [GO:0099052] References: PMID:21779028 Relationships: is a type of vesicle scission [GO:0099050]; is part of endocytosis [GO:0006897]